cell-cell signaling involved in pronephros development [GO:0039016] (biological process) Sources: GOC:mtg_kidney_jan10 Relationships: is a type of cell-cell signaling involved in kidney development [GO:0060995]; is part of pronephros development [GO:0048793] Also known as: cell-cell signaling involved in pronephric kidney development, cell-cell signalling involved in pronephros development Definition: Any process that mediates the transfer of information from one cell to another and contributes to the progression of the pronephros over time, from its formation to the mature organ.